{
  "gene_name": "Putative uncharacterized protein FLJ40140",
  "gene": "UniProtKB:Q8N814",
  "term_label": "Unknown molecular function",
  "term_id": "UNKNOWN:0001",
  "gene_symbol": "Q8N814"
}